{
  "term_label": "positive regulation of ERK1 and ERK2 cascade",
  "gene": "UniProtKB:P22455",
  "term_id": "GO:0070374",
  "gene_symbol": "FGFR4",
  "gene_name": "Fibroblast growth factor receptor 4"
}